UDP-L-rhamnose synthase activity [GO:0010280] (molecular function) References: PMID:14701918 Sources: MetaCyc:RXN-5482 Relationships: is a type of transferase activity [GO:0016740] Also known as: UDP-4-keto-6-deoxy-D-glucose 3,5-epimerase-4-reductase activity Definition: Catalysis of the reaction: UDP-D-glucose + NADPH + H+ = UDP-L-rhamnose + NADP+ + H2O.